{
  "gene_name": "Claudin-5",
  "gene_symbol": "CLDN5",
  "gene": "UniProtKB:O00501",
  "term_id": "GO:0005923",
  "term_label": "bicellular tight junction"
}